{
  "gene_symbol": "AGO2",
  "term_id": "GO:0003727",
  "gene_name": "Protein argonaute-2",
  "gene": "UniProtKB:Q9UKV8",
  "term_label": "single-stranded RNA binding"
}